{
  "term_id": "GO:0005391",
  "gene_symbol": "ATP1A2",
  "term_label": "P-type sodium:potassium-exchanging transporter activity",
  "gene": "UniProtKB:P50993",
  "gene_name": "Sodium_potassium-transporting ATPase subunit alpha-2"
}